{
  "gene_symbol": "SEMA3C",
  "term_id": "GO:0050919",
  "gene": "UniProtKB:Q99985",
  "gene_name": "Semaphorin-3C",
  "term_label": "negative chemotaxis"
}